{
  "term_label": "Unknown cellular component",
  "gene_name": "Homeobox protein Hox-C13",
  "gene_symbol": "HOXC13",
  "term_id": "UNKNOWN:0003",
  "gene": "UniProtKB:P31276"
}